regulation of timing of cell differentiation [GO:0048505] (biological process) Definition: The process controlling the activation and/or rate at which relatively unspecialized cells acquire specialized features. Any process that modulates the rate, frequency or extent of the XXX at a consistent predetermined time point during its development. Sources: GOC:bf, GOC:dph, GOC:jid, GOC:tb Also known as: timing of cell differentiation Relationships: is a type of regulation of development, heterochronic [GO:0040034]; is a type of regulation of cell differentiation [GO:0045595] Subtypes: inhibition of neuroepithelial cell differentiation [GO:0002085], regulation of timing of neuron differentiation [GO:0060164]